{
  "gene": "UniProtKB:P00480",
  "term_id": "GO:0005739",
  "gene_symbol": "OTC",
  "gene_name": "Ornithine transcarbamylase, mitochondrial",
  "term_label": "mitochondrion"
}